multiple synapse bouton, contacting multiple dendrites [GO:0150088] (cellular component) Definition: A single axon terminal bouton making contact onto two or more dendritic spines protruding from multiple dendrites. Also known as: MSB2, type 2 multi-synapse bouton, type 2 multi-synaptic bouton, type 2 multiple spine synapse bouton, type 2 multiple-synapse bouton, type 2 multisynapse bouton, type 2 multisynaptic bouton Relationships: is a type of GO:0150086 References: PMID:10586883, PMID:11248111, PMID:22028887, PMID:24487234, PMID:7482800, PMID:8366344 Sources: GOC:aruk, GOC:bc